{
  "gene": "UniProtKB:Q12972",
  "gene_symbol": "PPP1R8",
  "term_id": "GO:0004865",
  "term_label": "protein serine/threonine phosphatase inhibitor activity",
  "gene_name": "Nuclear inhibitor of protein phosphatase 1"
}